Group I intron splicing [GO:0000372] (BP) Note: Note that Group I introns are known to be found in a number of places: rRNA, mRNA, and tRNA in organelles of fungi, plants, and protists; tRNA and mRNA of bacteria and bacteriophage; rRNA of protists and fungi; and occasionally in mRNA of animal mitochondria (e.g. sea anemone). Relationships: is a type of RNA splicing, via transesterification reactions with guanosine as nucleophile [GO:0000376] Definition: The splicing of Group I introns. This occurs by a ribozymic mechanism where the intron sequence forms a distinct 3D structure, characteristic of Group I introns and involved in determining the locations of the splice sites (there do not appear to be consensus splice site sequences) as well as having a role in catalyzing the splicing reactions, though protein factors are also required in vivo. Splicing occurs by a series of two transesterification reactions, generally with exogenous guanosine as the initiating nucleophile. The intron is excised as a linear piece (though it may subsequently circularize). References: PMID:11377794 Sources: GOC:krc Also known as: mRNA splicing